{
  "gene_symbol": "ASTN2",
  "gene_name": "Astrotactin-2",
  "gene": "UniProtKB:O75129",
  "term_id": "GO:0016020",
  "term_label": "membrane"
}